programmed cell death [GO:0012501] (biological process) Sources: GOC:lr, GOC:mtg_apoptosis Note: Note that this term should be used to annotate gene products in the organism undergoing the programmed cell death. To annotate genes in another organism whose products modulate programmed cell death in a host organism, consider the term 'modulation by symbiont of host programmed cell death ; GO:0052040'. Also, note that 'programmed cell death ; GO:0012501' should be used to refer to instances of caspase-independent cell death mechanisms, in the absence of further indications on the process taking place. At present, caspase-independent cell death is not yet represented in GO due to the lack of consensus and in-depth research on the topic. 'programmed cell death ; GO:0012501' may also be used to annotate gene products in taxa where apoptosis as defined in GO:0006915 does not occur, such as plants. You may also consider these specific children: GO:0097468 'programmed cell death in response to reactive oxygen species' (with descendants GO:0010421 'hydrogen peroxide-mediated programmed cell death' and GO:0010343 'singlet oxygen-mediated programmed cell death'), and GO:0009626 'plant-type hypersensitive response' and its children. Regulation: regulated by regulation of programmed cell death [GO:0043067]; positively regulated by positive regulation of programmed cell death [GO:0043068]; negatively regulated by negative regulation of programmed cell death [GO:0043069] Definition: A process which begins when a cell receives an internal or external signal and activates a series of biochemical events (signaling pathway). The process ends with the death of the cell. Relationships: is a type of cell death [GO:0008219]; has part GO:0007165 Subtypes: autolysis [GO:0001896], apoptotic process [GO:0006915], programmed cell death involved in cell development [GO:0010623], symbiont-induced defense-related programmed cell death [GO:0034050], autophagic cell death [GO:0048102], GO:0070268, GO:0097300, programmed cell death in response to reactive oxygen species [GO:0097468], GO:0097707, pyroptotic cell death [GO:0141201], programmed cell death in response to retinoic acid [GO:0160059], cuproptosis [GO:0160119] Also known as: regulated cell death, caspase-independent cell death, non-apoptotic programmed cell death, nonapoptotic programmed cell death, PCD, RCD, caspase-independent apoptosis